{
  "gene_name": "Protein YIPF5",
  "gene_symbol": "YIPF5",
  "gene": "UniProtKB:Q969M3",
  "term_id": "GO:0060628",
  "term_label": "regulation of ER to Golgi vesicle-mediated transport"
}